{
  "gene_symbol": "RXFP1",
  "term_label": "adenylate cyclase-activating G protein-coupled receptor signaling pathway",
  "gene": "UniProtKB:Q9HBX9",
  "gene_name": "Relaxin receptor 1",
  "term_id": "GO:0007189"
}